jasmonic acid and ethylene-dependent systemic resistance [GO:0009861] (biological process) Also known as: jasmonic acid and ethene-dependent systemic resistance, jasmonic acid/ethylene-dependent systemic resistance Relationships: is a type of GO:0009611; is a type of defense response to symbiont [GO:0140546] References: PMID:10234273 Sources: GOC:jy Definition: The jasmonic acid and ethylene (ethene) dependent process that confers broad spectrum systemic resistance to disease in response to wounding or a pathogen.